negative regulation of chromatin binding [GO:0035562] (biological process) Relationships: is a type of negative regulation of binding [GO:0051100]; negatively regulates chromatin binding [GO:0003682] Definition: Any process that stops or reduces the frequency, rate or extent of chromatin binding. Chromatin binding is the selective interaction with chromatin, the network of fibers of DNA, protein, and sometimes RNA, that make up the chromosomes of the eukaryotic nucleus during interphase. References: PMID:20404130 Sources: GOC:bf